{
  "gene_symbol": "DEFB1",
  "gene": "UniProtKB:P60022",
  "gene_name": "Beta-defensin 1",
  "term_id": "GO:0005615",
  "term_label": "extracellular space"
}